{
  "gene_name": "Exonuclease V",
  "gene_symbol": "EXO5",
  "gene": "UniProtKB:Q9H790",
  "term_label": "interstrand cross-link repair",
  "term_id": "GO:0036297"
}